poly(3-hydroxyoctanoate) depolymerase activity [GO:0050527] (molecular function) Definition: Catalysis of the reaction: H2O + poly[(R)-3-hydroxyoctanoate](n) = poly[(R)-3-hydroxyoctanoate](x) + poly[(R)-3-hydroxyoctanoate](n-x); x is 1-5. Relationships: is a type of carboxylic ester hydrolase activity [GO:0052689] Also known as: PHA depolymerase activity, poly((R)-hydroxyalkanoic acid) depolymerase activity, poly(HA) depolymerase activity, poly[(R)-hydroxyalkanoic acid] depolymerase, PHO depolymerase activity, poly((R)-3-hydroxyoctanoate) hydrolase activity, poly(3HO) depolymerase activity, poly(HA(MCL)) depolymerase activity, poly(HAMCL) depolymerase activity, poly[(R)-3-hydroxyoctanoate] hydrolase activity, poly{oxycarbonyl[(R)-2-pentylethylene]} hydrolase activity Sources: EC:3.1.1.76, MetaCyc:3.1.1.76-RXN